{
  "gene_name": "USP6 N-terminal-like protein",
  "term_id": "GO:0048227",
  "gene_symbol": "USP6NL",
  "term_label": "plasma membrane to endosome transport",
  "gene": "UniProtKB:Q92738"
}